{
  "gene": "UniProtKB:Q02818",
  "term_id": "GO:0005509",
  "gene_name": "Nucleobindin-1",
  "gene_symbol": "NUCB1",
  "term_label": "calcium ion binding"
}